transcription preinitiation complex assembly [GO:0070897] (biological process) Sources: GOC:txnOH Also known as: transcription PIC biosynthesis, transcription PIC formation, transcriptional preinitiation complex formation, DNA-dependent transcriptional preinitiation complex assembly, DNA-templated transcriptional preinitiation complex assembly, bacterial-type RNA polymerase preinitiation complex assembly, bacterial-type RNA polymerase transcription PIC formation, bacterial-type RNA polymerase transcriptional preinitiation complex formation Relationships: is a type of protein-DNA complex assembly [GO:0065004]; is part of DNA-templated transcription initiation [GO:0006352] Subtypes: RNA polymerase I preinitiation complex assembly [GO:0001188], GO:0051123, RNA polymerase III preinitiation complex assembly [GO:0070898] Definition: The formation of a large multiprotein-DNA complex that self-assembles on gene promoter through the sequential recruitment of the general initiation factors that compose the preinitiation complex (PIC). The PIC engages the RNA polymerase on its DNA template strand and sparks polymerization of the first few RNA nucleotides.